regulation of ripoptosome assembly involved in necroptotic process [GO:1902442] (BP) Subtypes: negative regulation of ripoptosome assembly involved in necroptotic process [GO:1902443] Definition: Any process that modulates the frequency, rate or extent of ripoptosome assembly involved in a necroptotic process. Relationships: is a type of regulation of protein-containing complex assembly [GO:0043254]; regulates ripoptosome assembly involved in necroptotic process [GO:1901026] References: PMID:21052097 Sources: GOC:TermGenie, GOC:dph, GOC:mtg_apoptosis Also known as: regulation of ripoptosome assembly involved in necroptosis